{
  "gene_symbol": "C9orf152",
  "term_id": "UNKNOWN:0002",
  "gene": "UniProtKB:Q5JTZ5",
  "term_label": "Unknown biological process",
  "gene_name": "Uncharacterized protein C9orf152"
}